regulation of pre-tubular aggregate formation by cell-cell signaling [GO:0072043] (biological process) Definition: Any process that mediates the transfer of information from one cell to another that modulates the rate, frequency, or extent of pre-tubular aggregate formation. Pre-tubular aggregate formation is the cell adhesion process in which mesenchymal cells adhere to one another in the initial stages of the formation of the pre-tubular aggregate, the earliest recognizable structure of the kidney. Sources: GOC:mtg_kidney_jan10 Also known as: regulation of pre-tubular aggregate formation by cell-cell signalling Relationships: is a type of cell-cell signaling [GO:0007267]; is_a regulation of cell-cell adhesion [GO:0022407]; is a type of regulation of morphogenesis of an epithelium [GO:1905330]; regulates pre-tubular aggregate formation [GO:0072035]